{
  "gene_symbol": "CAPN3",
  "gene_name": "Calpain-3",
  "gene": "UniProtKB:P20807",
  "term_label": "proteolysis",
  "term_id": "GO:0006508"
}